{
  "gene_name": "Catenin alpha-2",
  "term_label": "catenin complex",
  "gene": "UniProtKB:P26232",
  "term_id": "GO:0016342",
  "gene_symbol": "CTNNA2"
}